{
  "gene_name": "Thyroid receptor-interacting protein 11",
  "term_label": "Golgi apparatus",
  "gene": "UniProtKB:Q15643",
  "gene_symbol": "TRIP11",
  "term_id": "GO:0005794"
}